FAD-dependent histone H3K9me/H3K9me2 demethylase activity [GO:0140685] (molecular function) Also known as: histone H3K9me demethylase activity, histone H3K9me2 demethylase activity, histone H3-di/monomethyl-lysine-9 FAD-dependent demethylase activity References: PMID:22473470 Relationships: is a type of oxidoreductase activity, acting on paired donors, with incorporation or reduction of molecular oxygen [GO:0016705]; is a type of histone H3K9 demethylase activity [GO:0032454] Definition: Catalysis of the removal of a methyl group from a di- or a monomethyl-lysine residue at position 9 of the histone H3 protein. This is a flavin adenine dinucleotide (FAD)-dependent amine oxidation reaction. Note: Comment: Note that the residue position corresponds to the canonical human H3 histone (UniProtKB:P84243); this residue is conserved across all eukaryotes. Residue 1 is the first residue following removal of the initiating Methionine (Met). Note that each histone is encoded by multiple genes, and sequences may vary across different genes within an organism.